{
  "term_id": "GO:0007186",
  "gene_name": "Olfactory receptor 5T1",
  "term_label": "G protein-coupled receptor signaling pathway",
  "gene": "UniProtKB:Q8NG75",
  "gene_symbol": "OR5T1"
}